{
  "gene": "UniProtKB:Q8TF50",
  "gene_symbol": "ZNF526",
  "term_label": "Unknown molecular function",
  "term_id": "UNKNOWN:0001",
  "gene_name": "Zinc finger protein 526"
}